{
  "term_label": "chromatin",
  "gene": "UniProtKB:Q6SJ93",
  "term_id": "GO:0000785",
  "gene_symbol": "FAM111B",
  "gene_name": "Serine protease FAM111B"
}